{
  "gene_name": "Transcriptional enhancer factor TEF-1",
  "term_id": "GO:0035329",
  "gene": "UniProtKB:P28347",
  "term_label": "hippo signaling",
  "gene_symbol": "TEAD1"
}